{
  "gene": "UniProtKB:Q9NUM3",
  "term_id": "UNKNOWN:0002",
  "term_label": "Unknown biological process",
  "gene_symbol": "SLC39A9",
  "gene_name": "Zinc transporter ZIP9"
}